{
  "gene_symbol": "CHRFAM7A",
  "term_label": "chemical synaptic transmission",
  "gene_name": "CHRNA7-FAM7A fusion protein",
  "gene": "UniProtKB:Q494W8",
  "term_id": "GO:0007268"
}